regulation of calcium ion import [GO:0090279] (biological process) Subtypes: GO:0090280, negative regulation of calcium ion import [GO:0090281], regulation of calcium ion import across plasma membrane [GO:1905664] Sources: GOC:BHF Also known as: regulation of transmembrane calcium influx Relationships: is a type of GO:0051924; regulates GO:0070509 Definition: Any process that modulates the rate, frequency, or extent of the directed movement of calcium ions into a cell or organelle.